extrinsic component of neuronal dense core vesicle membrane [GO:0098674] (cellular component) Relationships: is a type of extrinsic component of dense core granule membrane [GO:0098922]; is part of neuronal dense core vesicle membrane [GO:0099012] Definition: The component of the neuronal dense core vesicle membrane consisting of gene products and protein complexes that are loosely bound to one of its surfaces, but not integrated into the hydrophobic region. Sources: GOC:dos